{
  "term_id": "GO:0099175",
  "gene": "UniProtKB:Q7Z5H3",
  "gene_name": "Rho GTPase-activating protein 22",
  "term_label": "regulation of postsynapse organization",
  "gene_symbol": "ARHGAP22"
}